dichotomous subdivision of terminal units involved in mammary gland duct morphogenesis [GO:0060598] (biological process) Relationships: is a type of dichotomous subdivision of an epithelial terminal unit [GO:0060600]; BFO_0000050 GO:0060751 References: PMID:17120154 Sources: GOC:dph Definition: The process in which the terminal end of a mammary duct bifurcates. Also known as: primary mammary duct branching